{
  "gene": "UniProtKB:O75093",
  "term_label": "extracellular space",
  "term_id": "GO:0005615",
  "gene_symbol": "SLIT1",
  "gene_name": "Slit homolog 1 protein"
}